{
  "gene": "UniProtKB:Q9HBJ8",
  "gene_symbol": "CLTRN",
  "gene_name": "Collectrin",
  "term_label": "plasma membrane",
  "term_id": "GO:0005886"
}